{
  "gene_name": "Myelin protein zero-like protein 2",
  "term_id": "UNKNOWN:0001",
  "gene": "UniProtKB:O60487",
  "gene_symbol": "MPZL2",
  "term_label": "Unknown molecular function"
}